{
  "term_label": "protein insertion into mitochondrial outer membrane",
  "gene_name": "Metaxin-1",
  "gene": "UniProtKB:Q13505",
  "gene_symbol": "MTX1",
  "term_id": "GO:0045040"
}